{
  "gene": "UniProtKB:Q16678",
  "term_id": "GO:0042178",
  "gene_name": "Cytochrome P450 1B1",
  "gene_symbol": "CYP1B1",
  "term_label": "xenobiotic catabolic process"
}